{
  "gene_symbol": "H2BC14",
  "term_id": "GO:0061844",
  "gene": "UniProtKB:Q99879",
  "term_label": "antimicrobial humoral immune response mediated by antimicrobial peptide",
  "gene_name": "Histone H2B type 1-M"
}